{
  "term_label": "Unknown cellular component",
  "gene_symbol": "TRGJP1",
  "term_id": "UNKNOWN:0003",
  "gene_name": "T cell receptor gamma joining P1 (Fragment)",
  "gene": "UniProtKB:A0A0A0MT97"
}